{
  "term_label": "cell migration",
  "gene_name": "Glypican-1",
  "term_id": "GO:0016477",
  "gene": "UniProtKB:P35052",
  "gene_symbol": "GPC1"
}